{
  "gene_name": "Germinal-center associated nuclear protein",
  "gene_symbol": "MCM3AP",
  "gene": "UniProtKB:O60318",
  "term_label": "nucleus",
  "term_id": "GO:0005634"
}